{
  "gene_name": "Integrin alpha-V",
  "gene_symbol": "ITGAV",
  "term_label": "cell surface",
  "gene": "UniProtKB:P06756",
  "term_id": "GO:0009986"
}